{
  "term_label": "protein processing",
  "gene_name": "Presenilin-associated rhomboid-like protein, mitochondrial",
  "term_id": "GO:0016485",
  "gene_symbol": "PARL",
  "gene": "UniProtKB:Q9H300"
}